{
  "gene": "UniProtKB:Q9H7D0",
  "gene_name": "Dedicator of cytokinesis protein 5",
  "gene_symbol": "DOCK5",
  "term_id": "GO:0005085",
  "term_label": "guanyl-nucleotide exchange factor activity"
}